{
  "term_label": "structural constituent of nuclear pore",
  "gene_name": "Nuclear pore complex protein Nup98-Nup96",
  "gene": "UniProtKB:P52948",
  "term_id": "GO:0017056",
  "gene_symbol": "NUP98"
}